{
  "gene": "UniProtKB:Q96DB2",
  "term_label": "histone deacetylase complex",
  "gene_symbol": "HDAC11",
  "term_id": "GO:0000118",
  "gene_name": "Histone deacetylase 11"
}